{
  "term_label": "Unknown cellular component",
  "term_id": "UNKNOWN:0003",
  "gene_name": "G antigen 12G",
  "gene": "UniProtKB:P0CL81",
  "gene_symbol": "GAGE12G"
}